negative regulation of interleukin-19 production [GO:0032702] (biological process) Also known as: down regulation of interleukin-19 production, down-regulation of interleukin-19 production, downregulation of interleukin-19 production, negative regulation of IL-19 production, inhibition of interleukin-19 production, negative regulation of interleukin-19 biosynthetic process Relationships: is a type of GO:0001818; is a type of regulation of interleukin-19 production [GO:0032662]; RO_0002212 interleukin-19 production [GO:0032622] Sources: GOC:mah Definition: Any process that stops, prevents, or reduces the frequency, rate, or extent of interleukin-19 production.